{
  "gene_symbol": "CSF3R",
  "gene_name": "Granulocyte colony-stimulating factor receptor",
  "gene": "UniProtKB:Q99062",
  "term_id": "GO:0008284",
  "term_label": "positive regulation of cell population proliferation"
}